ammonium import across plasma membrane [GO:0140157] (biological process) References: PMID:16999738 Sources: GOC:vw Relationships: is a type of ammonium transmembrane transport [GO:0072488]; is a type of inorganic cation import across plasma membrane [GO:0098659] Definition: The directed movement of an ammonium ion from outside of a cell, across the plasma membrane and into the cytosol.